{
  "gene": "UniProtKB:Q8NFF5",
  "term_label": "FMN adenylyltransferase activity",
  "gene_name": "FAD synthase",
  "term_id": "GO:0003919",
  "gene_symbol": "FLAD1"
}